{
  "gene": "UniProtKB:O76021",
  "gene_symbol": "RSL1D1",
  "gene_name": "Ribosomal L1 domain-containing protein 1",
  "term_label": "RNA binding",
  "term_id": "GO:0003723"
}